{
  "gene_symbol": "CDC37",
  "gene": "UniProtKB:Q16543",
  "term_id": "GO:0006457",
  "term_label": "protein folding",
  "gene_name": "Hsp90 co-chaperone Cdc37"
}